{
  "term_label": "mitochondrial translation",
  "gene_symbol": "MRPL16",
  "gene_name": "Large ribosomal subunit protein uL16m",
  "term_id": "GO:0032543",
  "gene": "UniProtKB:Q9NX20"
}